{
  "term_id": "GO:0004749",
  "gene": "UniProtKB:P60891",
  "term_label": "ribose phosphate diphosphokinase activity",
  "gene_symbol": "PRPS1",
  "gene_name": "Ribose-phosphate pyrophosphokinase 1"
}